{
  "term_label": "Unknown molecular function",
  "gene_name": "Putative uncharacterized protein encoded by LINC00114",
  "gene_symbol": "LINC00114",
  "gene": "UniProtKB:Q6XXX2",
  "term_id": "UNKNOWN:0001"
}